omega-hydroxyceramide transacylase activity [GO:0106341] (molecular function) Relationships: is a type of acyltransferase activity, transferring groups other than amino-acyl groups [GO:0016747] References: PMID:28248318 Sources: RHEA:55264 Definition: Catalysis of the reaction: 1,2,3-tri-(9Z,12Z)-octadecadienoylglycerol + N-(30-hydroxytriacontanoyl)-sphing-4-enine = di-(9Z,12Z)-octadecadienoylglycerol + N-[30-(9Z,12Z-octadecadienoyloxy)-triacontanoyl]-sphing-4-enine.